{
  "gene_name": "Inhibin beta E chain",
  "term_id": "GO:0005125",
  "term_label": "cytokine activity",
  "gene_symbol": "INHBE",
  "gene": "UniProtKB:P58166"
}